{
  "term_id": "GO:0006511",
  "gene_name": "Kelch-like protein 25",
  "term_label": "ubiquitin-dependent protein catabolic process",
  "gene": "UniProtKB:Q9H0H3",
  "gene_symbol": "KLHL25"
}